selenium binding [GO:0008430] (molecular function) Definition: Binding to a selenium (Se) ion. Relationships: is a type of small molecule binding [GO:0036094] Sources: GOC:ai